{
  "term_id": "UNKNOWN:0002",
  "gene_symbol": "WDCP",
  "term_label": "Unknown biological process",
  "gene": "UniProtKB:Q9H6R7",
  "gene_name": "WD repeat and coiled-coil-containing protein"
}